{
  "term_id": "GO:0043533",
  "gene_name": "Astrotactin-2",
  "gene": "UniProtKB:O75129",
  "gene_symbol": "ASTN2",
  "term_label": "inositol 1,3,4,5 tetrakisphosphate binding"
}